{
  "gene": "UniProtKB:Q9Y623",
  "term_id": "GO:0032982",
  "term_label": "myosin filament",
  "gene_symbol": "MYH4",
  "gene_name": "Myosin-4"
}